{
  "gene": "UniProtKB:Q9Y5Y0",
  "term_label": "heme binding",
  "gene_symbol": "FLVCR1",
  "term_id": "GO:0020037",
  "gene_name": "Heme transporter FLVCR1"
}